steroid 21-monooxygenase activity [GO:0004509] (molecular function) Also known as: steroid 21-hydroxylase activity, cytochrome P450 CYP21A1, cytochrome p450 XXIA1 activity, 21-hydroxylase activity, steroid,hydrogen-donor:oxygen oxidoreductase (21-hydroxylating) Subtypes: 17-hydroxyprogesterone 21-hydroxylase activity [GO:0103069], progesterone 21-hydroxylase activity [GO:0106309] Definition: Catalysis of the reaction: A C(21) steroid + [reduced NADPH--hemoprotein reductase] + O2 = a 21-hydroxy-C(21)-steroid + [oxidized NADPH--hemoprotein reductase] + H2O. Sources: RHEA:65612 Relationships: is a type of steroid hydroxylase activity [GO:0008395]; is a type of oxidoreductase activity, acting on paired donors, with incorporation or reduction of molecular oxygen, reduced flavin or flavoprotein as one donor, and incorporation of one atom of oxygen [GO:0016712]